{
  "term_label": "magnesium ion binding",
  "gene": "UniProtKB:P78330",
  "gene_symbol": "PSPH",
  "term_id": "GO:0000287",
  "gene_name": "Phosphoserine phosphatase"
}